{
  "gene_symbol": "STX12",
  "term_id": "GO:0005484",
  "gene": "UniProtKB:Q86Y82",
  "gene_name": "Syntaxin-12",
  "term_label": "SNAP receptor activity"
}